{
  "gene_name": "Putative ATP synthase subunit g 2, mitochondrial",
  "term_label": "proton motive force-driven ATP synthesis",
  "gene": "UniProtKB:Q7Z4Y8",
  "gene_symbol": "ATP5MGL",
  "term_id": "GO:0015986"
}